{
  "term_label": "flagellated sperm motility",
  "term_id": "GO:0030317",
  "gene_symbol": "ROPN1B",
  "gene": "UniProtKB:Q9BZX4",
  "gene_name": "Ropporin-1B"
}